{
  "gene": "UniProtKB:O95989",
  "gene_name": "Diphosphoinositol polyphosphate phosphohydrolase 1",
  "gene_symbol": "NUDT3",
  "term_id": "GO:1901909",
  "term_label": "diadenosine hexaphosphate catabolic process"
}